{
  "gene_symbol": "C11orf68",
  "gene": "UniProtKB:Q9H3H3",
  "term_id": "UNKNOWN:0001",
  "gene_name": "UPF0696 protein C11orf68",
  "term_label": "Unknown molecular function"
}